{
  "gene_symbol": "EPO",
  "term_id": "GO:0030295",
  "gene": "UniProtKB:P01588",
  "term_label": "protein kinase activator activity",
  "gene_name": "Erythropoietin"
}